{
  "term_id": "GO:0051453",
  "term_label": "regulation of intracellular pH",
  "gene_name": "Sodium_hydrogen exchanger 4",
  "gene_symbol": "SLC9A4",
  "gene": "UniProtKB:Q6AI14"
}